{
  "gene_name": "Glycogen phosphorylase, muscle form",
  "gene": "UniProtKB:P11217",
  "term_id": "GO:0030170",
  "gene_symbol": "PYGM",
  "term_label": "pyridoxal phosphate binding"
}